host cell endoplasmic reticulum [GO:0044165] (cellular component) Also known as: host endoplasmic reticulum Relationships: is a type of host intracellular membrane-bounded organelle [GO:0033648]; is_a GO:0033655 Subtypes: host cell rough endoplasmic reticulum [GO:0044168], host cell smooth endoplasmic reticulum [GO:0044170] Definition: The irregular network of unit membranes, visible only by electron microscopy, that occurs in the host cell cytoplasm of many eukaryotic cells. The membranes form a complex meshwork of tubular channels, which are often expanded into slitlike cavities called cisternae. The host ER takes two forms, rough (or granular), with ribosomes adhering to the outer surface, and smooth (with no ribosomes attached). Sources: GOC:jl